3'-phosphoadenosine 5'-phosphosulfate metabolic process [GO:0050427] (biological process) Subtypes: 3'-phosphoadenosine 5'-phosphosulfate biosynthetic process [GO:0050428] Relationships: is a type of GO:0006790; is a type of purine ribonucleotide metabolic process [GO:0009150]; is a type of purine ribonucleoside bisphosphate metabolic process [GO:0034035]; is a type of oxoacid metabolic process [GO:0043436] Definition: The chemical reactions and pathways involving 3'-phosphoadenosine 5'-phosphosulfate, a naturally occurring mixed anhydride. It is an intermediate in the formation of a variety of sulfo compounds in biological systems. Sources: ISBN:0198506732 Also known as: 3'-phosphoadenosine 5'-phosphosulfate metabolism, 3'-phosphoadenosine 5'-phosphosulphate metabolic process, 3'-phosphoadenosine 5'-phosphosulphate metabolism, 3'-phosphoadenylyl-sulfate metabolic process, 3'-phosphoadenylyl-sulfate metabolism, PAPS metabolic process, PAPS metabolism, adenosine 3'-phosphate 5'-phosphosulfate metabolic process, adenosine 3'-phosphate 5'-phosphosulfate metabolism, phosphoadenosine phosphosulfate metabolic process, phosphoadenosine phosphosulfate metabolism